{
  "gene_name": "Myosin-13",
  "term_id": "GO:0000146",
  "gene_symbol": "MYH13",
  "gene": "UniProtKB:Q9UKX3",
  "term_label": "microfilament motor activity"
}